peptidyl-arginine deglycation [GO:0036527] (biological process) Definition: The removal of a sugar or dicarbonyl from an arginine residue of a glycated protein. References: PMID:14568004, PMID:25416785 Sources: GOC:PARL, GOC:bf Also known as: deglycation of N-acetylarginine Relationships: is a type of peptidyl-arginine modification [GO:0018195]; is_a protein deglycation [GO:0036525]